{
  "gene_name": "Interleukin-12 receptor subunit beta-1",
  "term_label": "receptor complex",
  "term_id": "GO:0043235",
  "gene": "UniProtKB:P42701",
  "gene_symbol": "IL12RB1"
}